{
  "term_id": "GO:0070166",
  "gene_name": "Amelogenin, Y isoform",
  "term_label": "enamel mineralization",
  "gene_symbol": "AMELY",
  "gene": "UniProtKB:Q99218"
}